calcium-dependent phospholipase C activity [GO:0050429] (molecular function) Relationships: is a type of phospholipase C activity [GO:0004629] References: PMID:25769297, PMID:9426125 Definition: Catalysis of the reaction: a phosphatidylcholine + H2O = 1,2-diacylglycerol + choline phosphate. This reaction requires Ca2+.